{
  "term_label": "extracellular space",
  "term_id": "GO:0005615",
  "gene_name": "Xanthine dehydrogenase_oxidase",
  "gene_symbol": "XDH",
  "gene": "UniProtKB:P47989"
}